basolateral cytoplasm [GO:0090652] (cellular component) Relationships: is_a cellular anatomical structure [GO:0110165]; is part of cytoplasm [GO:0005737] Definition: The region of the cytoplasm located at the basolateral side of the cell. Used in reference to animal polarized epithelial cells. References: PMID:17494872